{
  "term_id": "GO:0030139",
  "gene_symbol": "RIN3",
  "term_label": "endocytic vesicle",
  "gene_name": "Ras and Rab interactor 3",
  "gene": "UniProtKB:Q8TB24"
}